{
  "gene_symbol": "PPP6R1",
  "term_label": "protein phosphatase regulator activity",
  "gene": "UniProtKB:Q9UPN7",
  "gene_name": "Serine_threonine-protein phosphatase 6 regulatory subunit 1",
  "term_id": "GO:0019888"
}